{
  "gene": "UniProtKB:Q9HBE1",
  "term_label": "negative regulation of transcription by RNA polymerase II",
  "gene_name": "POZ-, AT hook-, and zinc finger-containing protein 1",
  "gene_symbol": "PATZ1",
  "term_id": "GO:0000122"
}